{
  "gene_name": "Acidic amino acid decarboxylase GADL1",
  "term_label": "Unknown biological process",
  "term_id": "UNKNOWN:0002",
  "gene": "UniProtKB:Q6ZQY3",
  "gene_symbol": "GADL1"
}